{
  "gene": "UniProtKB:Q17RR3",
  "term_label": "phospholipase A1 activity",
  "term_id": "GO:0008970",
  "gene_name": "Pancreatic lipase-related protein 3",
  "gene_symbol": "PNLIPRP3"
}